{
  "gene_name": "NF-X1-type zinc finger protein NFXL1",
  "term_label": "RNA polymerase II transcription regulatory region sequence-specific DNA binding",
  "gene_symbol": "NFXL1",
  "term_id": "GO:0000977",
  "gene": "UniProtKB:Q6ZNB6"
}